regulation of acetate catabolic process [GO:0045734] (biological process) Definition: Any process that modulates the frequency, rate or extent of the chemical reactions and pathways resulting in the breakdown of acetate, the anion of acetic acid. Relationships: is_a regulation of catabolic process [GO:0009894]; is a type of regulation of ketone metabolic process [GO:0010565]; is a type of regulation of small molecule metabolic process [GO:0062012]; regulates acetate catabolic process [GO:0045733] Sources: GOC:go_curators Subtypes: GO:0045753, GO:0045754 Also known as: regulation of acetate breakdown, regulation of acetate catabolism, regulation of acetate degradation